neuroligin family protein binding [GO:0097109] (molecular function) References: PMID:21424692 Sources: GOC:BHF, GOC:pr, GOC:sjp Definition: Binding to a member of the neuroligin protein family, neuronal cell surface proteins that mediate synapse formation. Relationships: is a type of signaling receptor binding [GO:0005102]